zygotene [GO:0000238] (biological process) Relationships: is_a meiosis I cell cycle phase [GO:0098764]; is part of meiotic prophase I [GO:0007128] Sources: GOC:mtg_cell_cycle Note: Note that this term should not be used for direct annotation. If you are trying to make an annotation to x phase, it is likely that the correct annotation is 'regulation of x/y phase transition' or to a process which occurs during the reported phase (i.e mitotic DNA replication for mitotic S-phase). To capture the phase when a specific location or process is observed, the phase term can be used in an annotation extension (PMID:24885854) applied to a cellular component term (with the relation exists_during) or a biological process term (with the relation happens_during). Definition: The cell cycle phase which follows leptotene during prophase I of meiosis, and during which each chromosome pairs with its homolog; the two become aligned and crossing over may occur.